{
  "gene": "UniProtKB:P29558",
  "term_id": "GO:0008266",
  "gene_name": "RNA-binding motif, single-stranded-interacting protein 1",
  "gene_symbol": "RBMS1",
  "term_label": "poly(U) RNA binding"
}